antibiotic biosynthetic process [GO:0017000] (biological process) Relationships: is a type of GO:0009058; is a type of GO:0016999 Also known as: antibiotic anabolism, antibiotic biosynthesis, antibiotic formation, antibiotic synthesis Subtypes: phenazine biosynthetic process [GO:0002047], aminoglycoside antibiotic biosynthetic process [GO:0030648], peptide antibiotic biosynthetic process [GO:0030651], GO:0030654, macrolide biosynthetic process [GO:0033068], puromycin biosynthetic process [GO:0043638], GO:0043642, GO:0043644, enniatin biosynthetic process [GO:0046585], mycophenolic acid biosynthetic process [GO:0140722] Sources: GOC:go_curators Definition: The chemical reactions and pathways resulting in the formation of an antibiotic, a substance produced by or derived from certain fungi, bacteria, and other organisms, that can destroy or inhibit the growth of other microorganisms.